{
  "gene": "UniProtKB:Q53H12",
  "gene_symbol": "AGK",
  "term_id": "GO:0005737",
  "gene_name": "Acylglycerol kinase, mitochondrial",
  "term_label": "cytoplasm"
}